{
  "gene_symbol": "GIGYF1",
  "term_label": "Unknown molecular function",
  "term_id": "UNKNOWN:0001",
  "gene": "UniProtKB:O75420",
  "gene_name": "GRB10-interacting GYF protein 1"
}